{
  "gene": "UniProtKB:Q99676",
  "gene_name": "Zinc finger protein 184",
  "term_label": "RNA polymerase II cis-regulatory region sequence-specific DNA binding",
  "term_id": "GO:0000978",
  "gene_symbol": "ZNF184"
}